{
  "gene_name": "Forkhead box protein D4-like 3",
  "term_id": "GO:0009653",
  "gene": "UniProtKB:Q6VB84",
  "gene_symbol": "FOXD4L3",
  "term_label": "anatomical structure morphogenesis"
}